regulation of apoptotic cell clearance [GO:2000425] (biological process) Relationships: is a type of regulation of phagocytosis [GO:0050764]; regulates GO:0043277 Sources: GOC:obol Subtypes: negative regulation of apoptotic cell clearance [GO:2000426], GO:2000427 Also known as: regulation of apoptotic cell removal, regulation of efferocytosis, regulation of programmed cell clearance Definition: Any process that modulates the frequency, rate or extent of apoptotic cell clearance.